{
  "gene": "UniProtKB:Q9Y4X3",
  "gene_symbol": "CCL27",
  "term_id": "GO:0071222",
  "term_label": "cellular response to lipopolysaccharide",
  "gene_name": "C-C motif chemokine 27"
}